{
  "gene_symbol": "Q8N9P0",
  "term_label": "Unknown biological process",
  "gene_name": "Putative uncharacterized protein FLJ36797",
  "gene": "UniProtKB:Q8N9P0",
  "term_id": "UNKNOWN:0002"
}